{
  "gene_symbol": "RGSL1",
  "gene": "UniProtKB:A5PLK6",
  "term_label": "Unknown cellular component",
  "gene_name": "Regulator of G-protein signaling protein-like",
  "term_id": "UNKNOWN:0003"
}